{
  "term_id": "GO:0032456",
  "term_label": "endocytic recycling",
  "gene_name": "Vacuolar protein sorting-associated protein 51 homolog",
  "gene": "UniProtKB:Q9UID3",
  "gene_symbol": "VPS51"
}